{
  "gene_symbol": "TRIM62",
  "gene": "UniProtKB:Q9BVG3",
  "term_id": "GO:0043123",
  "term_label": "positive regulation of canonical NF-kappaB signal transduction",
  "gene_name": "E3 ubiquitin-protein ligase TRIM62"
}